{
  "term_label": "killing of cells of another organism",
  "term_id": "GO:0031640",
  "gene_name": "Statherin",
  "gene_symbol": "STATH",
  "gene": "UniProtKB:P02808"
}